{
  "term_id": "GO:0004674",
  "gene_symbol": "TAOK2",
  "term_label": "protein serine/threonine kinase activity",
  "gene_name": "Serine_threonine-protein kinase TAO2",
  "gene": "UniProtKB:Q9UL54"
}